{
  "gene_name": "Uncharacterized protein C14orf28",
  "term_label": "Unknown cellular component",
  "gene": "UniProtKB:Q4W4Y0",
  "term_id": "UNKNOWN:0003",
  "gene_symbol": "DORIP1"
}